parthenolide synthase activity [GO:0102626] (molecular function) Definition: Catalysis of the reaction: (+)-costunolide + O2 + reduced [NADPH--hemoprotein reductase] = H+ + H2O + oxidized [NADPH--hemoprotein reductase] + parthenolide. Sources: RHEA:61320 Relationships: is a type of GO:0016712